positive regulation of peripheral T cell tolerance induction [GO:0002851] (biological process) Definition: Any process that activates or increases the frequency, rate, or extent of peripheral T cell tolerance induction. Also known as: up regulation of peripheral T cell tolerance induction, up-regulation of peripheral T cell tolerance induction, upregulation of peripheral T cell tolerance induction, activation of peripheral T cell tolerance induction, stimulation of peripheral T cell tolerance induction Relationships: is a type of positive regulation of peripheral tolerance induction [GO:0002660]; is a type of GO:0002666; is a type of GO:0002711; is a type of regulation of peripheral T cell tolerance induction [GO:0002849]; positively regulates GO:0002458 Subtypes: positive regulation of T cell tolerance induction to tumor cell [GO:0002848] Sources: GOC:add